{
  "term_label": "osteoclast differentiation",
  "gene_name": "Protein strawberry notch homolog 2",
  "term_id": "GO:0030316",
  "gene": "UniProtKB:Q9Y2G9",
  "gene_symbol": "SBNO2"
}